{
  "gene": "UniProtKB:Q9BX46",
  "term_label": "mRNA stabilization",
  "gene_name": "RNA-binding protein 24",
  "gene_symbol": "RBM24",
  "term_id": "GO:0048255"
}